{
  "term_id": "GO:0007417",
  "gene_name": "Metal regulatory transcription factor 1",
  "gene": "UniProtKB:Q14872",
  "term_label": "central nervous system development",
  "gene_symbol": "MTF1"
}